regulation of testosterone secretion [GO:2000843] (biological process) Subtypes: GO:2000844, positive regulation of testosterone secretion [GO:2000845] Sources: GOC:sl Definition: Any process that modulates the frequency, rate or extent of testosterone secretion. Relationships: is a type of regulation of lipid transport [GO:0032368]; is_a regulation of hormone secretion [GO:0046883]; regulates testosterone secretion [GO:0035936]